{
  "term_label": "bicarbonate transport",
  "gene": "UniProtKB:P04920",
  "gene_symbol": "SLC4A2",
  "gene_name": "Anion exchange protein 2",
  "term_id": "GO:0015701"
}